glutathione specific gamma-glutamylcyclotransferase activity [GO:0061928] (molecular function) Relationships: is a type of amidine-lyase activity [GO:0016842] References: PMID:23070364, PMID:27913623 Definition: Catalysis of the reaction: glutathione = 5-oxoproline + L-cysteinylglycine.